regulation of response to acetate [GO:1901457] (biological process) Relationships: is a type of regulation of response to stimulus [GO:0048583]; regulates response to acetate [GO:0010034] Sources: GOC:TermGenie, GOC:mengo_curators Subtypes: negative regulation of response to acetate [GO:1901458], GO:1901459 Definition: Any process that modulates the frequency, rate or extent of response to acetate.